{
  "term_id": "GO:0003746",
  "gene_symbol": "EEF1A1P5",
  "term_label": "translation elongation factor activity",
  "gene_name": "Putative elongation factor 1-alpha-like 3",
  "gene": "UniProtKB:Q5VTE0"
}